{
  "term_label": "intermediate filament",
  "gene_name": "Neurofilament light polypeptide",
  "term_id": "GO:0005882",
  "gene": "UniProtKB:P07196",
  "gene_symbol": "NEFL"
}